negative regulation of cardiac ventricle formation [GO:1904943] (biological process) Also known as: down regulation of cardiac ventricle formation, down-regulation of cardiac ventricle formation, downregulation of cardiac ventricle formation, inhibition of cardiac ventricle formation Relationships: is a type of negative regulation of cardiac chamber formation [GO:1901211]; is a type of negative regulation of cardiac ventricle development [GO:1904413]; is a type of GO:1904942; negatively regulates cardiac ventricle formation [GO:0003211] References: PMID:23575307 Sources: GOC:BHF, GOC:BHF_miRNA, GOC:TermGenie, GOC:bc, GO_REF:0000058 Definition: Any process that stops, prevents or reduces the frequency, rate or extent of cardiac ventricle formation.